regulation of telomerase RNA localization to Cajal body [GO:1904872] (BP) Definition: Any process that modulates the frequency, rate or extent of telomerase RNA localization to Cajal body. Relationships: is a type of regulation of localization [GO:0032879]; RO_0002211 telomerase RNA localization to Cajal body [GO:0090671] References: PMID:25467444 Sources: GOC:BHF, GOC:BHF_telomere, GOC:TermGenie, GOC:nc, GO_REF:0000058 Subtypes: GO:1904873, positive regulation of telomerase RNA localization to Cajal body [GO:1904874]